{
  "gene": "UniProtKB:Q5EBL8",
  "term_label": "neurotransmitter secretion",
  "gene_symbol": "PDZD11",
  "term_id": "GO:0007269",
  "gene_name": "PDZ domain-containing protein 11"
}